lagging strand elongation [GO:0006273] (biological process) Subtypes: mitotic DNA replication lagging strand elongation [GO:1903459] Sources: GOC:mah, ISBN:071673706X, ISBN:0815316194 Relationships: is a type of DNA strand elongation involved in DNA replication [GO:0006271]; has part DNA replication, synthesis of primer [GO:0006269]; has part DNA replication, removal of RNA primer [GO:0043137] Definition: The process in which an existing DNA strand is extended in a net 3' to 5' direction by activities including the addition of nucleotides to the 3' end of the strand, complementary to an existing template, as part of DNA replication. Lagging strand DNA elongation proceeds by discontinuous synthesis of short stretches of DNA, known as Okazaki fragments, from RNA primers; these fragments are then joined by DNA ligase. Although each segment of nascent DNA is synthesized in the 5' to 3' direction, the overall direction of lagging strand synthesis is 3' to 5', mirroring the progress of the replication fork.